{
  "term_label": "signaling receptor activity",
  "gene_name": "Leucine-rich repeat-containing protein 3C",
  "gene": "UniProtKB:A6NJW4",
  "gene_symbol": "LRRC3C",
  "term_id": "GO:0038023"
}